RNA polymerase II transcription regulatory region sequence-specific DNA binding [GO:0000977] (molecular function) Also known as: RNA polymerase II regulatory region DNA binding Relationships: is a type of transcription cis-regulatory region binding [GO:0000976] Regulation: RO_0002211 by regulation of RNA polymerase II regulatory region sequence-specific DNA binding [GO:1903025]; negatively regulated by negative regulation of RNA polymerase II regulatory region sequence-specific DNA binding [GO:1903026] Subtypes: RNA polymerase II cis-regulatory region sequence-specific DNA binding [GO:0000978], RNA polymerase II core promoter sequence-specific DNA binding [GO:0000979], RNA polymerase II intronic transcription regulatory region sequence-specific DNA binding [GO:0001162] Sources: GOC:txnOH Note: To minimize ambiguity in the use of the word "promoter" in GO, we have chosen the phrase "transcription regulatory region" to refer to all of the regulatory regions. Regulatory regions in the DNA which control initiation may include the "core promoter" where the basal transcription machinery binds, the "core promoter proximal region" where regulatory factors other than the basal machinery bind. There are also additional regulatory regions, in both the DNA and the RNA transcript, which regulate elongation or termination of transcription. Definition: Binding to a specific sequence of DNA that is part of a regulatory region that controls the transcription of a gene or cistron by RNA polymerase II.